{
  "gene": "UniProtKB:Q9UNH6",
  "gene_symbol": "SNX7",
  "gene_name": "Sorting nexin-7",
  "term_id": "GO:0061709",
  "term_label": "reticulophagy"
}